{
  "gene_symbol": "DPYS",
  "term_id": "GO:0004157",
  "gene": "UniProtKB:Q14117",
  "term_label": "dihydropyrimidinase activity",
  "gene_name": "Dihydropyrimidinase"
}